{
  "gene": "UniProtKB:O15162",
  "term_label": "plasma membrane",
  "gene_symbol": "PLSCR1",
  "gene_name": "Phospholipid scramblase 1",
  "term_id": "GO:0005886"
}